{
  "gene_symbol": "MS4A14",
  "term_label": "plasma membrane",
  "gene_name": "Membrane-spanning 4-domains subfamily A member 14",
  "gene": "UniProtKB:Q96JA4",
  "term_id": "GO:0005886"
}